{
  "gene_symbol": "RHOQ",
  "gene_name": "Rho-related GTP-binding protein RhoQ",
  "term_id": "GO:0007165",
  "term_label": "signal transduction",
  "gene": "UniProtKB:P17081"
}